{
  "gene_symbol": "ITGBL1",
  "gene": "UniProtKB:O95965",
  "term_label": "cell-matrix adhesion",
  "gene_name": "Integrin beta-like protein 1",
  "term_id": "GO:0007160"
}